{
  "gene": "UniProtKB:Q53EL9",
  "gene_name": "Seizure protein 6 homolog",
  "gene_symbol": "SEZ6",
  "term_label": "dendritic shaft",
  "term_id": "GO:0043198"
}